{
  "gene": "UniProtKB:P06280",
  "term_label": "alpha-galactosidase activity",
  "gene_symbol": "GLA",
  "gene_name": "Alpha-galactosidase A",
  "term_id": "GO:0004557"
}